{
  "term_label": "Unknown molecular function",
  "gene_symbol": "SLC35F4",
  "gene_name": "Solute carrier family 35 member F4",
  "term_id": "UNKNOWN:0001",
  "gene": "UniProtKB:A4IF30"
}